{
  "gene_name": "Cytosolic endo-beta-N-acetylglucosaminidase",
  "gene": "UniProtKB:Q8NFI3",
  "term_label": "N-glycan processing",
  "term_id": "GO:0006491",
  "gene_symbol": "ENGASE"
}